positive regulation of isotype switching [GO:0045830] (biological process) Also known as: positive regulation of class switch recombination, positive regulation of class switching, positive regulation of isotype switch recombination, up regulation of isotype switching, up-regulation of isotype switching, upregulation of isotype switching, activation of isotype switching, stimulation of isotype switching Sources: GOC:go_curators Subtypes: positive regulation of isotype switching to IgE isotypes [GO:0048295], positive regulation of isotype switching to IgA isotypes [GO:0048298], positive regulation of isotype switching to IgD isotypes [GO:0048301], positive regulation of isotype switching to IgG isotypes [GO:0048304] Relationships: is a type of positive regulation of immunoglobulin production [GO:0002639]; is a type of GO:0002891; is a type of regulation of isotype switching [GO:0045191]; is a type of GO:0045911; is a type of GO:0050871; is a type of GO:0051094; positively regulates isotype switching [GO:0045190] Definition: Any process that activates or increases the frequency, rate or extent of isotype switching.